forebrain anterior/posterior pattern specification [GO:0021797] (biological process) Definition: The creation of specific areas of progenitor domains along the anterior-posterior axis of the developing forebrain. Sources: GOC:cls, GOC:dgh, GOC:dph, GOC:jid, GO_REF:0000021 Relationships: is a type of anterior/posterior pattern specification [GO:0009952]; is part of forebrain regionalization [GO:0021871] Also known as: forebrain anterior-posterior pattern specification